{
  "term_id": "GO:0071526",
  "gene_name": "Semaphorin-4F",
  "gene": "UniProtKB:O95754",
  "gene_symbol": "SEMA4F",
  "term_label": "semaphorin-plexin signaling pathway"
}